{
  "gene_name": "Monocarboxylate transporter 14",
  "gene": "UniProtKB:Q7RTX9",
  "term_label": "carboxylic acid transmembrane transport",
  "gene_symbol": "SLC16A14",
  "term_id": "GO:1905039"
}